{
  "gene_symbol": "CSMD3",
  "term_id": "UNKNOWN:0003",
  "term_label": "Unknown cellular component",
  "gene": "UniProtKB:Q7Z407",
  "gene_name": "CUB and sushi domain-containing protein 3"
}